negative regulation of actin filament bundle assembly [GO:0032232] (biological process) Relationships: is a type of regulation of actin filament bundle assembly [GO:0032231]; is a type of GO:0051494; is a type of negative regulation of supramolecular fiber organization [GO:1902904]; RO_0002212 actin filament bundle assembly [GO:0051017] Subtypes: negative regulation of stress fiber assembly [GO:0051497], GO:0090339 Also known as: down regulation of actin filament bundle formation, down-regulation of actin filament bundle formation, downregulation of actin filament bundle formation, inhibition of actin filament bundle formation Definition: Any process that stops, prevents, or reduces the frequency, rate or extent of the assembly of actin filament bundles. Sources: GOC:mah